{
  "term_label": "regulation of transcription by RNA polymerase II",
  "gene_symbol": "ZNF697",
  "term_id": "GO:0006357",
  "gene": "UniProtKB:Q5TEC3",
  "gene_name": "Zinc finger protein 697"
}